{
  "gene": "UniProtKB:Q8IU89",
  "term_id": "GO:0005783",
  "gene_symbol": "CERS3",
  "term_label": "endoplasmic reticulum",
  "gene_name": "Ceramide synthase 3"
}